{
  "term_label": "neutral L-amino acid transmembrane transporter activity",
  "gene_symbol": "SLC1A5",
  "gene": "UniProtKB:Q15758",
  "term_id": "GO:0015175",
  "gene_name": "Neutral amino acid transporter B(0)"
}